{
  "gene": "UniProtKB:A6NDH6",
  "term_id": "UNKNOWN:0002",
  "gene_name": "Olfactory receptor 5H15",
  "term_label": "Unknown biological process",
  "gene_symbol": "OR5H15"
}